{
  "term_id": "GO:1901897",
  "term_label": "regulation of relaxation of cardiac muscle",
  "gene_symbol": "AKAP6",
  "gene": "UniProtKB:Q13023",
  "gene_name": "A-kinase anchor protein 6"
}